{
  "term_label": "nucleoplasm",
  "gene": "UniProtKB:Q9HCD5",
  "gene_name": "Nuclear receptor coactivator 5",
  "term_id": "GO:0005654",
  "gene_symbol": "NCOA5"
}